{
  "term_id": "UNKNOWN:0002",
  "gene": "UniProtKB:Q5TEZ5",
  "gene_symbol": "C6orf163",
  "gene_name": "Uncharacterized protein C6orf163",
  "term_label": "Unknown biological process"
}